{
  "gene": "UniProtKB:Q05397",
  "term_label": "regulation of cell adhesion",
  "gene_name": "Focal adhesion kinase 1",
  "gene_symbol": "PTK2",
  "term_id": "GO:0030155"
}